{
  "gene_name": "Keratin, type II cuticular Hb2",
  "gene": "UniProtKB:Q9NSB4",
  "term_label": "keratinization",
  "term_id": "GO:0031424",
  "gene_symbol": "KRT82"
}